signal recognition particle, plasma membrane targeting [GO:0048501] (cellular component) Relationships: is a type of GO:0048500 Definition: A complex consisting of a protein and RNA component which binds the signal sequence of some proteins and facilitates their export to or across the plasma membrane. Sources: GOC:mlg, GOC:mtg_sensu